{
  "term_id": "UNKNOWN:0001",
  "gene_name": "Prickle-like protein 2",
  "gene": "UniProtKB:Q7Z3G6",
  "gene_symbol": "PRICKLE2",
  "term_label": "Unknown molecular function"
}